{
  "gene": "UniProtKB:Q9BYG8",
  "gene_symbol": "GSDMC",
  "term_label": "phosphatidylinositol-4-phosphate binding",
  "gene_name": "Gasdermin-C",
  "term_id": "GO:0070273"
}